{
  "gene_name": "Jhy protein homolog",
  "term_label": "Unknown cellular component",
  "term_id": "UNKNOWN:0003",
  "gene": "UniProtKB:Q6NUN7",
  "gene_symbol": "JHY"
}